{
  "gene": "UniProtKB:Q8N3E9",
  "term_label": "phosphatidylinositol-4,5-bisphosphate phospholipase C activity",
  "gene_symbol": "PLCD3",
  "term_id": "GO:0004435",
  "gene_name": "1-phosphatidylinositol 4,5-bisphosphate phosphodiesterase delta-3"
}